{
  "gene_name": "Zinc finger protein 471",
  "term_label": "nucleus",
  "term_id": "GO:0005634",
  "gene_symbol": "ZNF471",
  "gene": "UniProtKB:Q9BX82"
}